{
  "term_id": "GO:0007030",
  "gene_symbol": "UBXN2B",
  "gene": "UniProtKB:Q14CS0",
  "gene_name": "UBX domain-containing protein 2B",
  "term_label": "Golgi organization"
}